{
  "gene": "UniProtKB:O95238",
  "term_label": "cell differentiation",
  "term_id": "GO:0030154",
  "gene_name": "SAM pointed domain-containing Ets transcription factor",
  "gene_symbol": "SPDEF"
}